{
  "gene_symbol": "NPHP3",
  "gene_name": "Nephrocystin-3",
  "term_id": "GO:0097543",
  "term_label": "ciliary inversin compartment",
  "gene": "UniProtKB:Q7Z494"
}